{
  "term_id": "GO:0004930",
  "gene": "UniProtKB:P48145",
  "term_label": "G protein-coupled receptor activity",
  "gene_name": "Neuropeptides B_W receptor type 1",
  "gene_symbol": "NPBWR1"
}